astrocyte activation involved in immune response [GO:0002265] (biological process) Definition: A change in the morphology or behavior of an astrocyte resulting from exposure to an activating factor such as a cellular or soluble ligand, leading to the initiation or perpetuation of an immune response. Relationships: is a type of cell activation involved in immune response [GO:0002263]; is a type of GO:0048143 Also known as: astrocyte activation during immune response References: PMID:11138785 Sources: GOC:add